{
  "term_label": "regulation of transcription by RNA polymerase II",
  "gene_name": "Pancreas transcription factor 1 subunit alpha",
  "gene_symbol": "PTF1A",
  "term_id": "GO:0006357",
  "gene": "UniProtKB:Q7RTS3"
}